negative regulation of leukocyte adhesion to vascular endothelial cell [GO:1904995] (biological process) Subtypes: GO:1903237, negative regulation of leukocyte adhesion to arterial endothelial cell [GO:1904998] Definition: Any process that stops, prevents or reduces the frequency, rate or extent of leukocyte adhesion to vascular endothelial cell. Relationships: is a type of negative regulation of leukocyte cell-cell adhesion [GO:1903038]; is a type of regulation of leukocyte adhesion to vascular endothelial cell [GO:1904994]; negatively regulates leukocyte adhesion to vascular endothelial cell [GO:0061756] References: PMID:23897866 Sources: GOC:BHF, GOC:BHF_miRNA, GOC:TermGenie, GOC:bc, GO_REF:0000058 Also known as: down regulation of leukocyte adhesion to vascular endothelial cell, down-regulation of leukocyte adhesion to vascular endothelial cell, downregulation of leukocyte adhesion to vascular endothelial cell, inhibition of leukocyte adhesion to vascular endothelial cell